{
  "term_label": "plasma membrane",
  "term_id": "GO:0005886",
  "gene_symbol": "CLCN1",
  "gene": "UniProtKB:P35523",
  "gene_name": "Chloride channel protein 1"
}